{
  "gene": "UniProtKB:P53803",
  "gene_name": "DNA-directed RNA polymerases I, II, and III subunit RPABC4",
  "gene_symbol": "POLR2K",
  "term_id": "UNKNOWN:0002",
  "term_label": "Unknown biological process"
}